{
  "term_label": "G protein-coupled receptor activity",
  "gene_symbol": "TAS1R3",
  "gene_name": "Taste receptor type 1 member 3",
  "term_id": "GO:0004930",
  "gene": "UniProtKB:Q7RTX0"
}